{
  "gene": "UniProtKB:Q9NR63",
  "gene_name": "Cytochrome P450 26B1",
  "term_id": "UNKNOWN:0003",
  "term_label": "Unknown cellular component",
  "gene_symbol": "CYP26B1"
}